{
  "term_label": "Unknown cellular component",
  "term_id": "UNKNOWN:0003",
  "gene_symbol": "SLC7A5",
  "gene_name": "Large neutral amino acids transporter small subunit 1",
  "gene": "UniProtKB:Q01650"
}